growth hormone receptor complex [GO:0070195] (cellular component) Definition: A receptor complex that consists of two identical subunits and binds growth hormone. References: PMID:11445442 Sources: GOC:BHF, GOC:mah, GOC:vk Relationships: is a type of receptor complex [GO:0043235]